{
  "term_id": "GO:0000796",
  "gene_name": "Structural maintenance of chromosomes protein 4",
  "term_label": "condensin complex",
  "gene": "UniProtKB:Q9NTJ3",
  "gene_symbol": "SMC4"
}